IKKalpha-IKKalpha complex [GO:0038059] (cellular component) Relationships: is a type of GO:0032991 Definition: A homodimeric protein complex containing two IkappaB kinase (IKK) alpha subunits. Also known as: IKKalpha homodimer, IKKalpha homodimeric complex, IKKalpha-IKKalpha protein complex, IkappaB kinase alpha homodimer, IkappaB kinase-alpha homodimer References: PMID:18626576, PMID:21173796 Sources: GOC:bf